{
  "gene_name": "ADP-ribosylation factor-like protein 14",
  "term_id": "GO:0005737",
  "gene_symbol": "ARL14",
  "term_label": "cytoplasm",
  "gene": "UniProtKB:Q8N4G2"
}